{
  "term_label": "nucleoplasm",
  "gene_symbol": "TNRC6C",
  "term_id": "GO:0005654",
  "gene_name": "Trinucleotide repeat-containing gene 6C protein",
  "gene": "UniProtKB:Q9HCJ0"
}